{
  "term_label": "Unknown molecular function",
  "gene_symbol": "PXMP2",
  "gene_name": "Peroxisomal membrane protein 2",
  "term_id": "UNKNOWN:0001",
  "gene": "UniProtKB:Q9NR77"
}